{
  "gene_symbol": "FHOD3",
  "gene_name": "FH1_FH2 domain-containing protein 3",
  "gene": "UniProtKB:Q2V2M9",
  "term_label": "positive regulation of stress fiber assembly",
  "term_id": "GO:0051496"
}